{
  "term_label": "heart development",
  "gene_name": "Transforming growth factor beta-1 proprotein",
  "gene_symbol": "TGFB1",
  "term_id": "GO:0007507",
  "gene": "UniProtKB:P01137"
}